positive regulation of lateral mesodermal cell fate specification [GO:0048379] (biological process) Definition: Any process that activates or increases the frequency, rate or extent of lateral mesoderm cell fate specification. Sources: GOC:jid Also known as: positive regulation of lateral plate mesodermal cell fate specification, up regulation of lateral mesodermal cell fate specification, up-regulation of lateral mesodermal cell fate specification, upregulation of lateral mesodermal cell fate specification, activation of lateral mesodermal cell fate specification, stimulation of lateral mesodermal cell fate specification Relationships: is a type of GO:0048337; is a type of regulation of lateral mesodermal cell fate specification [GO:0048378]; positively regulates lateral mesodermal cell fate specification [GO:0048377]